{
  "term_id": "GO:0006357",
  "gene": "UniProtKB:Q96BV0",
  "term_label": "regulation of transcription by RNA polymerase II",
  "gene_symbol": "ZNF775",
  "gene_name": "Zinc finger protein 775"
}